[3-methyl-2-oxobutanoate dehydrogenase (acetyl-transferring)] kinase activity [GO:0047323] (molecular function) Sources: RHEA:17301 Also known as: [3-methyl-2-oxobutanoate dehydrogenase (lipoamide)] kinase activity, 3-methyl-2-oxobutanoate dehydrogenase (acetyl-transferring) kinase activity, ATP:3-methyl-2-oxobutanoate dehydrogenase (acetyl-transferring) phosphotransferase activity, BCK, BCKD kinase activity, BCODH kinase activity, STK2, branched-chain 2-oxo acid dehydrogenase kinase activity, branched-chain alpha-ketoacid dehydrogenase kinase activity, branched-chain keto acid dehydrogenase kinase activity, branched-chain oxo acid dehydrogenase kinase (phosphorylating) activity Definition: Catalysis of the reaction: ATP + L-seryl-[3-methyl-2-oxobutanoate dehydrogenase] = ADP + H+ + O-phospho-L-seryl-[3-methyl-2-oxobutanoate dehydrogenase]. Relationships: is a type of GO:0004674